{
  "term_label": "nucleus",
  "gene": "UniProtKB:P17035",
  "term_id": "GO:0005634",
  "gene_name": "Zinc finger protein 28",
  "gene_symbol": "ZNF28"
}